{
  "term_label": "receptor recycling",
  "gene_symbol": "PHETA2",
  "term_id": "GO:0001881",
  "gene_name": "Sesquipedalian-2",
  "gene": "UniProtKB:Q6ICB4"
}